corticotropin hormone secreting cell differentiation [GO:0060128] (biological process) Relationships: is a type of GO:0030154; is part of adenohypophysis development [GO:0021984] Definition: The process in which a relatively unspecialized cell acquires specialized structural and/or functional features of a corticotropic hormone secreting cell. An corticotropic hormone secreting cell is a basophil cell of the anterior pituitary that produces corticotropin. Sources: GOC:dph Also known as: adrenocorticotrophic hormone secreting cell differentiation, adrenocorticotropic hormone secreting cell differentiation, corticotrope differentiation, corticotroph differentiation, corticotrophin hormone secreting cell differentiation